{
  "gene_name": "Alpha-enolase",
  "term_label": "phosphopyruvate hydratase activity",
  "gene": "UniProtKB:P06733",
  "gene_symbol": "ENO1",
  "term_id": "GO:0004634"
}